{
  "gene_name": "Pre-mRNA-processing factor 6",
  "gene_symbol": "PRPF6",
  "term_label": "Unknown molecular function",
  "gene": "UniProtKB:O94906",
  "term_id": "UNKNOWN:0001"
}